{
  "gene_symbol": "RNF111",
  "term_label": "cytoplasm",
  "gene_name": "E3 ubiquitin-protein ligase Arkadia",
  "term_id": "GO:0005737",
  "gene": "UniProtKB:Q6ZNA4"
}